regulation of epinephrine uptake [GO:0051626] (biological process) Subtypes: negative regulation of epinephrine uptake [GO:0051627], positive regulation of epinephrine uptake [GO:0051628] Also known as: regulation of adrenaline uptake, regulation of epinephrine import Definition: Any process that modulates the frequency, rate or extent of the directed movement of the neurotransmitter epinephrine into a cell. Sources: GOC:ai Relationships: is a type of regulation of transport [GO:0051049]; RO_0002211 epinephrine uptake [GO:0051625]